negative regulation of DNA replication initiation involved in plasmid copy number maintenance [GO:0060910] (BP) Relationships: is_a GO:0032297; is a type of regulation of DNA replication initiation involved in plasmid copy number maintenance [GO:0060909] Definition: Any process that decreases the frequency, rate or extent of initiation of plasmid DNA replication that contributes to copy number maintenance. Sources: GOC:dph, GOC:tb